{
  "gene": "UniProtKB:A6NDN8",
  "term_id": "UNKNOWN:0001",
  "gene_name": "Putative ubiquitin-like protein FUBI-like protein ENSP00000310146",
  "term_label": "Unknown molecular function",
  "gene_symbol": "A6NDN8"
}